{
  "gene_symbol": "IRF2BPL",
  "term_label": "Unknown molecular function",
  "term_id": "UNKNOWN:0001",
  "gene_name": "Probable E3 ubiquitin-protein ligase IRF2BPL",
  "gene": "UniProtKB:Q9H1B7"
}